{
  "gene": "UniProtKB:P01709",
  "term_id": "UNKNOWN:0001",
  "gene_name": "Immunoglobulin lambda variable 2-8",
  "gene_symbol": "IGLV2-8",
  "term_label": "Unknown molecular function"
}